N-cyclopropylmelamine catabolic process [GO:0042202] (biological process) Definition: The chemical reactions and pathways resulting in the breakdown of N-cyclopropylmelamine, a triazine compound commonly used as an insecticide. Relationships: is_a s-triazine compound catabolic process [GO:0042204] Also known as: N-cyclopropylmelamine breakdown, N-cyclopropylmelamine catabolism, N-cyclopropylmelamine degradation, cyromazine catabolic process, cyromazine catabolism Sources: UM-BBD_pathwayID:cpm